methyltransferase cap2 activity [GO:0120550] (molecular function) Relationships: is a type of GO:0008171; is a type of RNA methyltransferase activity [GO:0008173] Definition: Catalysis of the reaction: a 5'-end (N(7)-methyl 5'-triphosphoguanosine)-(2'-O-methyl-ribonucleoside)-(ribonucleotide) in mRNA or snRNA + S-adenosyl-L-methionine = a 5'-end (N(7)-methyl 5'-triphosphoguanosine)-(2'-O-methyl-ribonucleoside)-(2'-O-methyl-ribonucleotide) in mRNA or snRNA + S-adenosyl-L-homocysteine + H+. This activity catalyzes the methylation of the ribose on the second transcribed nucleotide of mRNAs and snRNAs. Also known as: cap2-MTase activity, mRNA (nucleoside-2'-O-)-methyltransferase activity Sources: EC:2.1.1.296